trans-Golgi network transport vesicle [GO:0030140] (cellular component) Relationships: is a type of Golgi-associated vesicle [GO:0005798]; is a type of GO:0030133; is a type of clathrin-coated vesicle [GO:0030136] Definition: A vesicle that mediates transport between the trans-Golgi network and other parts of the cell. Also known as: TGN transport vesicle, trans-Golgi network constitutive secretory pathway transport vesicle Sources: GOC:mah